{
  "term_id": "GO:0017121",
  "gene_symbol": "PLSCR3",
  "gene_name": "Phospholipid scramblase 3",
  "gene": "UniProtKB:Q9NRY6",
  "term_label": "plasma membrane phospholipid scrambling"
}